{
  "term_label": "snRNA binding",
  "gene_name": "RNA-binding motif protein, X-linked-like-2",
  "gene_symbol": "RBMXL2",
  "term_id": "GO:0017069",
  "gene": "UniProtKB:O75526"
}